{
  "term_id": "GO:0042721",
  "term_label": "TIM22 mitochondrial import inner membrane insertion complex",
  "gene_name": "Mitochondrial import inner membrane translocase subunit Tim29",
  "gene_symbol": "TIMM29",
  "gene": "UniProtKB:Q9BSF4"
}